response to injury involved in regulation of muscle adaptation [GO:0014876] (biological process) Definition: Any process that results in a change in state or activity of a cell or an organism (in terms of movement, secretion, enzyme production, gene expression, etc.) as a result of a injury. This process occurs as part of the regulation of muscle adaptation. Also known as: response to injury involved in regulation of muscle plasticity Subtypes: GO:0014885 Relationships: is a type of response to wounding [GO:0009611]; is a type of response to stimulus involved in regulation of muscle adaptation [GO:0014874] Sources: GOC:ef, GOC:mtg_muscle